{
  "gene_name": "Tyrosine-protein phosphatase non-receptor type 5",
  "term_id": "GO:0030054",
  "gene_symbol": "PTPN5",
  "gene": "UniProtKB:P54829",
  "term_label": "cell junction"
}